{
  "gene_name": "Serine_threonine-protein kinase PAK 4",
  "gene_symbol": "PAK4",
  "term_label": "cellular response to starvation",
  "gene": "UniProtKB:O96013",
  "term_id": "GO:0009267"
}